{
  "gene_name": "Tubulin-specific chaperone D",
  "term_label": "microtubule cytoskeleton organization",
  "gene_symbol": "TBCD",
  "term_id": "GO:0000226",
  "gene": "UniProtKB:Q9BTW9"
}